{
  "gene_symbol": "HIPK2",
  "term_id": "GO:0005634",
  "gene_name": "Homeodomain-interacting protein kinase 2",
  "gene": "UniProtKB:Q9H2X6",
  "term_label": "nucleus"
}